{
  "gene_symbol": "CLIP2",
  "term_id": "GO:0031122",
  "term_label": "cytoplasmic microtubule organization",
  "gene_name": "CAP-Gly domain-containing linker protein 2",
  "gene": "UniProtKB:Q9UDT6"
}